{
  "term_label": "Unknown biological process",
  "gene": "UniProtKB:Q8N7A1",
  "term_id": "UNKNOWN:0002",
  "gene_name": "Kelch domain-containing protein 1",
  "gene_symbol": "KLHDC1"
}